{
  "gene_name": "Complement C1q tumor necrosis factor-related protein 5",
  "term_label": "plasma membrane",
  "term_id": "GO:0005886",
  "gene": "UniProtKB:Q9BXJ0",
  "gene_symbol": "C1QTNF5"
}